sebaceous gland development [GO:0048733] (biological process) Subtypes: GO:1903699 Sources: GOC:jid Definition: The process whose specific outcome is the progression of the sebaceous gland over time, from its formation to the mature structure. Relationships: is a type of gland development [GO:0048732]; is part of skin development [GO:0043588]